{
  "gene_symbol": "SULF2",
  "term_label": "N-acetylglucosamine-6-sulfatase activity",
  "term_id": "GO:0008449",
  "gene": "UniProtKB:Q8IWU5",
  "gene_name": "Extracellular sulfatase Sulf-2"
}